glycerol dehydrogenase (acceptor) activity [GO:0047955] (MF) Sources: EC:1.1.99.22, RHEA:17493 Also known as: glycerol:(acceptor) 1-oxidoreductase activity, glycerol:acceptor 1-oxidoreductase activity Relationships: is a type of GO:0016614 Definition: Catalysis of the reaction: A + glycerol = AH(2) + glycerone.